{
  "gene_symbol": "HOXA1",
  "term_label": "RNA polymerase II cis-regulatory region sequence-specific DNA binding",
  "gene_name": "Homeobox protein Hox-A1",
  "term_id": "GO:0000978",
  "gene": "UniProtKB:P49639"
}